{
  "term_label": "neuron differentiation",
  "gene_name": "Protein Wnt-8b",
  "term_id": "GO:0030182",
  "gene_symbol": "WNT8B",
  "gene": "UniProtKB:Q93098"
}